integrin alphaM-beta2 complex [GO:0034688] (cellular component) References: PMID:12297042 Also known as: alphaM-beta2 integrin complex, Itgam-Itgb2 complex Relationships: is a type of integrin complex [GO:0008305] Definition: An integrin complex that comprises one alphaM subunit and one beta2 subunit.